{
  "gene_symbol": "ARL9",
  "term_id": "UNKNOWN:0001",
  "term_label": "Unknown molecular function",
  "gene": "UniProtKB:Q6T311",
  "gene_name": "ADP-ribosylation factor-like protein 9"
}